{
  "term_label": "nucleus",
  "gene_name": "Heat shock factor protein 1",
  "gene_symbol": "HSF1",
  "gene": "UniProtKB:Q00613",
  "term_id": "GO:0005634"
}